D-xylulose reductase activity [GO:0046526] (molecular function) Definition: Catalysis of the reaction: NAD+ + xylitol = D-xylulose + H+ + NADH. Also known as: xylitol dehydrogenase activity Sources: RHEA:20433 Relationships: is a type of GO:0016616; is a type of hexitol dehydrogenase activity [GO:0031320]